{
  "gene_symbol": "CCDC107",
  "gene": "UniProtKB:Q8WV48",
  "term_id": "UNKNOWN:0001",
  "gene_name": "Coiled-coil domain-containing protein 107",
  "term_label": "Unknown molecular function"
}